{
  "term_id": "UNKNOWN:0001",
  "term_label": "Unknown molecular function",
  "gene_symbol": "TRAJ48",
  "gene_name": "T cell receptor alpha joining 48 (Fragment)",
  "gene": "UniProtKB:A0A075B6V3"
}